{
  "term_id": "GO:0000122",
  "gene_symbol": "DNAJB1",
  "term_label": "negative regulation of transcription by RNA polymerase II",
  "gene": "UniProtKB:P25685",
  "gene_name": "DnaJ homolog subfamily B member 1"
}